{
  "term_label": "nucleus",
  "gene_symbol": "SWT1",
  "term_id": "GO:0005634",
  "gene": "UniProtKB:Q5T5J6",
  "gene_name": "Transcriptional protein SWT1"
}